{
  "term_id": "GO:0046470",
  "gene_name": "Phospholipase A2 group V",
  "term_label": "phosphatidylcholine metabolic process",
  "gene_symbol": "PLA2G5",
  "gene": "UniProtKB:P39877"
}